{
  "gene_name": "Serine_threonine-protein kinase TAO3",
  "term_label": "protein serine/threonine kinase activity",
  "term_id": "GO:0004674",
  "gene": "UniProtKB:Q9H2K8",
  "gene_symbol": "TAOK3"
}